cytokinin transport [GO:0010184] (biological process) Definition: The directed movement of cytokinins, a class of adenine-derived compounds that can function in plants as growth regulators, into, out of or within a cell, or between cells, by means of some agent such as a transporter or pore. Sources: GOC:lr Relationships: is a type of hormone transport [GO:0009914]